{
  "gene": "UniProtKB:O15204",
  "term_id": "UNKNOWN:0003",
  "term_label": "Unknown cellular component",
  "gene_name": "ADAM DEC1",
  "gene_symbol": "ADAMDEC1"
}